{
  "gene": "UniProtKB:Q92982",
  "gene_symbol": "NINJ1",
  "term_id": "GO:0005886",
  "gene_name": "Ninjurin-1",
  "term_label": "plasma membrane"
}